{
  "term_label": "structural constituent of ribosome",
  "gene": "UniProtKB:P27635",
  "gene_symbol": "RPL10",
  "term_id": "GO:0003735",
  "gene_name": "Large ribosomal subunit protein uL16"
}